{
  "term_id": "GO:0031640",
  "gene_symbol": "DEFB118",
  "gene_name": "Defensin beta 118",
  "gene": "UniProtKB:Q96PH6",
  "term_label": "killing of cells of another organism"
}